{
  "gene_symbol": "C4orf51",
  "gene_name": "Uncharacterized protein C4orf51",
  "gene": "UniProtKB:C9J302",
  "term_label": "Unknown biological process",
  "term_id": "UNKNOWN:0002"
}